{
  "gene": "UniProtKB:Q9UPR5",
  "gene_name": "Sodium_calcium exchanger 2",
  "term_id": "GO:0006874",
  "term_label": "intracellular calcium ion homeostasis",
  "gene_symbol": "SLC8A2"
}